RNA polymerase I core promoter sequence-specific DNA binding [GO:0001164] (molecular function) Also known as: RNA polymerase I CORE element sequence-specific DNA binding, RNA polymerase I CORE element sequence-specific DNA binding transcription factor recruiting transcription factor activity, transcription factor activity, RNA polymerase I CORE element binding transcription factor recruiting References: PMID:12865296, PMID:14969726, PMID:8057832 Sources: GOC:txnOH Relationships: is a type of core promoter sequence-specific DNA binding [GO:0001046]; is a type of RNA polymerase I transcription regulatory region sequence-specific DNA binding [GO:0001163]; is part of RNA polymerase I preinitiation complex assembly [GO:0001188] Definition: Binding to a regulatory region composed of the transcription start site and binding sites for transcription factors of the RNA polymerase I transcription machinery. This site is often referred to as the CORE element. In mammalian cells, the CORE element functions in conjunction with the Upstream Control Element (UCE), while in fungi, protozoa, and plants, the CORE element functions without a UCE.